instar larval development [GO:0002168] (biological process) Relationships: is a type of larval development [GO:0002164]; is a type of instar larval or pupal development [GO:0002165] Sources: GOC:bf, GOC:mtg_sensu Definition: The process whose specific outcome is the progression of the larva over time, from its formation to the mature structure. This begins with the newly hatched first-instar larva, through its maturation to the end of the last larval stage. An example of this process is found in Drosophila melanogaster.